{
  "gene_symbol": "HSD17B7",
  "term_label": "cholesterol biosynthetic process",
  "gene": "UniProtKB:P56937",
  "term_id": "GO:0006695",
  "gene_name": "3-keto-steroid reductase_17-beta-hydroxysteroid dehydrogenase 7"
}